{
  "term_id": "GO:0015464",
  "term_label": "acetylcholine receptor activity",
  "gene_symbol": "CHRNE",
  "gene": "UniProtKB:Q04844",
  "gene_name": "Acetylcholine receptor subunit epsilon"
}